negative regulation of R8 cell differentiation [GO:0045680] (biological process) Also known as: down regulation of R8 differentiation, down-regulation of R8 differentiation, downregulation of R8 differentiation, negative regulation of R8 differentiation, inhibition of R8 differentiation Relationships: is a type of regulation of R8 cell differentiation [GO:0045679]; is a type of negative regulation of compound eye photoreceptor cell differentiation [GO:0110118]; negatively regulates R8 cell differentiation [GO:0045465] Sources: GOC:dph, GOC:go_curators, GOC:tb Definition: Any process that stops, prevents, or reduces the frequency, rate or extent of R8 cell differentiation.